host cell synapse [GO:0044221] (cellular component) Relationships: is a type of host cell part [GO:0033643] Sources: GOC:rph Definition: The junction between a nerve fiber of one host neuron and another host neuron or muscle fiber or glial cell; the site of interneuronal communication.